arbuscule [GO:0085041] (cellular component) Relationships: is a type of GO:0085035 Definition: Highly branched symbiont haustoria within host root cortex cells, responsible for nutrient exchange. Note: See also: periarbuscular membrane ; GO:0085042. Sources: GOC:pamgo_curators